regulation of ATP citrate synthase activity [GO:2000983] (biological process) Definition: Any process that modulates the frequency, rate or extent of ATP citrate synthase activity. Sources: GOC:BHF Also known as: regulation of ATP citrate (pro-S)-lyase activity, regulation of ATP-citrate (pro-S)-lyase activity, regulation of ATP-citrate (pro-S-)-lyase activity, regulation of ATP-citric lyase activity, regulation of ATP:citrate oxaloacetate-lyase ((pro-S)-CH(2)COO(-)->acetyl-CoA) (ATP- dephosphorylating) activity, regulation of acetyl-CoA:oxaloacetate acetyltransferase (isomerizing; ADP- phosphorylating) activity, regulation of acetyl-CoA:oxaloacetate acetyltransferase (isomerizing; ADP-phosphorylating), regulation of adenosine triphosphate citrate lyase activity, regulation of citrate-ATP lyase activity, regulation of ATP:citrate oxaloacetate-lyase [(pro-S)-CH2COO-rightacetyl-CoA] (ATP-dephosphorylating), regulation of acetyl-CoA:oxaloacetate C-acetyltransferase [(pro-S)-carboxymethyl-forming, ADP-phosphorylating], regulation of citrate cleavage enzyme activity, regulation of citric cleavage enzyme activity Relationships: is a type of regulation of transferase activity [GO:0051338]; regulates ATP citrate synthase activity [GO:0003878]